{
  "term_id": "GO:0005737",
  "gene": "UniProtKB:Q16851",
  "term_label": "cytoplasm",
  "gene_symbol": "UGP2",
  "gene_name": "UTP--glucose-1-phosphate uridylyltransferase"
}